{
  "gene": "UniProtKB:Q9H257",
  "gene_name": "Caspase recruitment domain-containing protein 9",
  "term_id": "GO:0035591",
  "term_label": "signaling adaptor activity",
  "gene_symbol": "CARD9"
}